nuclear import signal receptor activity [GO:0061608] (molecular function) Definition: Combining with a nuclear import signal (NIS) on a cargo to be transported, to mediate transport of the cargo through the nuclear pore, from the cytoplasm to the nuclear lumen. The cargo can be either a RNA or a protein. References: PMID:28713609 Sources: GOC:dph, GOC:pg, GOC:vw, Wikipedia:Nuclear_transport Also known as: importin activity Relationships: is a type of nucleocytoplasmic carrier activity [GO:0140142]; is part of import into nucleus [GO:0051170]